{
  "term_label": "G-protein beta-subunit binding",
  "gene_symbol": "GNGT1",
  "term_id": "GO:0031681",
  "gene": "UniProtKB:P63211",
  "gene_name": "Guanine nucleotide-binding protein G(T) subunit gamma-T1"
}